{
  "gene": "UniProtKB:Q8IUB5",
  "gene_name": "WAP four-disulfide core domain protein 13",
  "term_id": "GO:0045087",
  "gene_symbol": "WFDC13",
  "term_label": "innate immune response"
}